{
  "gene_name": "Protein mono-ADP-ribosyltransferase PARP10",
  "gene": "UniProtKB:Q53GL7",
  "term_label": "nucleus",
  "term_id": "GO:0005634",
  "gene_symbol": "PARP10"
}